ecgonone methyl ester catabolic process [GO:1901871] (biological process) Definition: The chemical reactions and pathways resulting in the breakdown of ecgonone methyl ester. Relationships: is a type of alkaloid catabolic process [GO:0009822]; is a type of ketone catabolic process [GO:0042182] Also known as: ecgonone methyl ester breakdown, ecgonone methyl ester catabolism, ecgonone methyl ester degradation References: PMID:22665766 Sources: GOC:TermGenie